{
  "term_id": "UNKNOWN:0003",
  "term_label": "Unknown cellular component",
  "gene": "UniProtKB:Q8N8C0",
  "gene_name": "Zinc finger protein 781",
  "gene_symbol": "ZNF781"
}